{
  "gene_name": "Homeobox protein notochord",
  "term_id": "GO:0000978",
  "gene_symbol": "NOTO",
  "gene": "UniProtKB:A8MTQ0",
  "term_label": "RNA polymerase II cis-regulatory region sequence-specific DNA binding"
}